{
  "term_id": "UNKNOWN:0001",
  "gene_symbol": "CFAP57",
  "gene": "UniProtKB:Q96MR6",
  "gene_name": "Cilia- and flagella-associated protein 57",
  "term_label": "Unknown molecular function"
}